{
  "gene_name": "Zinc finger and BTB domain-containing protein 14",
  "term_label": "nucleoplasm",
  "gene": "UniProtKB:O43829",
  "term_id": "GO:0005654",
  "gene_symbol": "ZBTB14"
}